{
  "term_label": "Unknown biological process",
  "term_id": "UNKNOWN:0002",
  "gene": "UniProtKB:Q6ZUB1",
  "gene_symbol": "SPATA31E1",
  "gene_name": "Spermatogenesis-associated protein 31E1"
}